{
  "gene_symbol": "PRXL2B",
  "term_id": "GO:0001516",
  "gene_name": "Prostamide_prostaglandin F synthase",
  "term_label": "prostaglandin biosynthetic process",
  "gene": "UniProtKB:Q8TBF2"
}